{
  "gene_name": "Zinc finger imprinted 3",
  "gene": "UniProtKB:Q96PE6",
  "term_label": "DNA-binding transcription factor activity, RNA polymerase II-specific",
  "term_id": "GO:0000981",
  "gene_symbol": "ZIM3"
}